{
  "gene_symbol": "CHRNA2",
  "gene_name": "Neuronal acetylcholine receptor subunit alpha-2",
  "term_label": "acetylcholine receptor signaling pathway",
  "gene": "UniProtKB:Q15822",
  "term_id": "GO:0095500"
}